somatic processes downstream of sex determination signal [GO:0007546] (biological process) Relationships: is_a processes downstream of sex determination signal [GO:0007545] Definition: The events determining the somatic sexual phenotype after the initial transmission of that phenotype to soma-specific information pathways. Sources: GOC:ems